{
  "term_label": "transmembrane transporter binding",
  "term_id": "GO:0044325",
  "gene": "UniProtKB:Q13303",
  "gene_name": "Voltage-gated potassium channel subunit beta-2",
  "gene_symbol": "KCNAB2"
}